protein C-terminal leucine carboxyl O-methyltransferase activity [GO:0018423] (molecular function) References: PMID:8514774 Definition: Catalysis of the reaction: S-adenosyl-L-methionine + [protein]-L-leucine = S-adenosyl-L-homocysteine + [protein]-L-leucine methyl ester. This modification occurs only at the oxygen atoms of the free alpha carboxyl group of a leucine residue at the C-terminus of the protein. Also known as: protein-leucine O-methyltransferase activity, protein phosphatase methyltransferase activity Relationships: is a type of protein C-terminal carboxyl O-methyltransferase activity [GO:0003880]; is a type of S-adenosylmethionine-dependent methyltransferase activity [GO:0008757]